{
  "term_label": "innate immune response",
  "term_id": "GO:0045087",
  "gene_name": "Tripartite motif-containing protein 43",
  "gene_symbol": "TRIM43",
  "gene": "UniProtKB:Q96BQ3"
}